lipid hydroxylation [GO:0002933] (biological process) Also known as: fatty acid hydroxylation Definition: The covalent attachment of a hydroxyl group to one or more fatty acids in a lipid. References: PMID:15658937 Sources: GOC:hjd Relationships: is a type of GO:0030258